{
  "term_label": "Unknown cellular component",
  "term_id": "UNKNOWN:0003",
  "gene": "UniProtKB:A0A024R1R8",
  "gene_symbol": "TMA7B",
  "gene_name": "Translation machinery-associated protein 7B"
}